{
  "term_label": "NADH pyrophosphatase activity",
  "term_id": "GO:0035529",
  "gene_name": "NAD-capped RNA hydrolase NUDT12",
  "gene": "UniProtKB:Q9BQG2",
  "gene_symbol": "NUDT12"
}